snoRNA binding [GO:0030515] (molecular function) Relationships: is a type of RNA binding [GO:0003723] Subtypes: GO:0034511, box C/D sno(s)RNA binding [GO:0034512], box H/ACA snoRNA binding [GO:0034513] Definition: Binding to a small nucleolar RNA. Sources: GOC:mah